{
  "gene_name": "Cyclin-K",
  "gene": "UniProtKB:O75909",
  "term_id": "GO:0032786",
  "gene_symbol": "CCNK",
  "term_label": "positive regulation of DNA-templated transcription, elongation"
}